quinate O-hydroxycinnamoyltransferase activity [GO:0047205] (molecular function) Definition: Catalysis of the reaction: feruloyl-CoA + quinate = O-feruloylquinate + CoA. Also known as: feruloyl-CoA:quinate O-(hydroxycinnamoyl)transferase activity, hydroxycinnamoyl coenzyme A-quinate transferase activity Sources: EC:2.3.1.99, MetaCyc:2.3.1.99-RXN Relationships: is a type of GO:0050737